protein-containing complex assembly [GO:0065003] (biological process) Also known as: cellular protein complex assembly, cellular macromolecule complex assembly, cellular protein-containing complex assembly, chaperone activity, macromolecular complex assembly, macromolecule complex assembly, protein complex assembly, protein complex formation Regulation: negatively regulated by negative regulation of protein-containing complex assembly [GO:0031333]; positively regulated by positive regulation of protein-containing complex assembly [GO:0031334]; regulated by regulation of protein-containing complex assembly [GO:0043254] Definition: The aggregation, arrangement and bonding together of a set of macromolecules to form a protein-containing complex. Relationships: is a type of cellular component assembly [GO:0022607]; is a type of protein-containing complex organization [GO:0043933] Subtypes: GO:0000921, protein-DNA-RNA complex assembly [GO:0001116], exocyst assembly [GO:0001927], MHC protein complex assembly [GO:0002396], GO:0002501, steroid hormone receptor complex assembly [GO:0006463], SRP-dependent cotranslational protein targeting to membrane, signal sequence recognition [GO:0006617], tubulin complex assembly [GO:0007021], activation of transmembrane receptor protein tyrosine kinase activity [GO:0007171], GO:0007172, GO:0007181, GO:0010207, GO:0010257, SCF complex assembly [GO:0010265], GO:0010275, COP9 signalosome assembly [GO:0010387], synaptic vesicle priming [GO:0016082], cytochrome complex assembly [GO:0017004], GO:0018419, protein-RNA complex assembly [GO:0022618], myosin filament assembly [GO:0031034], post-translational protein targeting to membrane, docking [GO:0031203], GO:0033108, GO:0033622, respiratory chain complex II assembly [GO:0034552], GO:0035493, GO:0036034, SAGA complex assembly [GO:0036285], TCR signalosome assembly [GO:0036399], nodal receptor complex assembly [GO:0038099], dosage compensation complex assembly [GO:0042714], proteasome assembly [GO:0043248], starch utilization system complex assembly [GO:0044574], GO:0046931, GO:0048195, Golgi membrane coat protein complex assembly [GO:0048197], GO:0048208, clathrin coat assembly [GO:0048268], photosystem I assembly [GO:0048564], chaperone-mediated protein complex assembly [GO:0051131], protein polymerization [GO:0051258], GO:0051259, kinetochore assembly [GO:0051382], GO:0061789, LinE complex assembly [GO:0062120], radial spoke assembly [GO:0062177], protein-DNA complex assembly [GO:0065004], protein-lipid complex assembly [GO:0065005], proton-transporting two-sector ATPase complex assembly [GO:0070071], GO:0070096, GO:0070196, GO:0070217, GO:0070286, voltage-gated calcium channel complex assembly [GO:0070978], death-inducing signaling complex assembly [GO:0071550], podosome assembly [GO:0071800], Mre11 complex assembly [GO:0072685], MCM complex assembly [GO:0072689], protein-containing complex assembly involved in synapse maturation [GO:0090126], DNA repair complex assembly [GO:0090735], eukaryotic translation initiation factor 4F complex assembly [GO:0097010], GO:0097314, ripoptosome assembly [GO:0097343], ribulose bisphosphate carboxylase complex assembly [GO:0110102], mRNA cleavage and polyadenylation specificity factor complex assembly [GO:0110105], MBF transcription complex assembly [GO:0120185], ciliary centrin arm assembly [GO:0120273], canonical inflammasome complex assembly [GO:0140632], GO:0140970, non-canonical inflammasome complex assembly [GO:0160075], GO:0160234, sodium-translocating NADH-quinone reductase complex assembly [GO:0160293], gamma-tubulin complex assembly [GO:1902481], GO:1902561, GO:1902605, exon-exon junction complex assembly [GO:1903040], GO:1903359, VCP-NPL4-UFD1 AAA ATPase complex assembly [GO:1904210], pyroptosome complex assembly [GO:1904270], Wnt-Frizzled-LRP5/6 complex assembly [GO:1904701], Atg1/ULK1 kinase complex assembly [GO:1904745], chaperone-mediated autophagy translocation complex assembly [GO:1904763], anaphase-promoting complex assembly [GO:1904824], beta-catenin-TCF complex assembly [GO:1904837], beta-catenin destruction complex assembly [GO:1904885], Wnt signalosome assembly [GO:1904887], GO:1904895, eukaryotic translation initiation factor 2 complex assembly [GO:1905143], GO:1905173, Y-shaped link assembly [GO:1905350], ciliary necklace assembly [GO:1905352], GO:1905353, FACT complex assembly [GO:1905635], GO:1905660, TORC1 complex assembly [GO:1905669], RNA polymerase I assembly [GO:1990113], RNA polymerase II core complex assembly [GO:1990114], RNA polymerase III assembly [GO:1990115], Dsc E3 ubiquitin ligase complex assembly [GO:1990155] Sources: GOC:jl